{
  "term_id": "UNKNOWN:0001",
  "gene_symbol": "SMIM32",
  "gene": "UniProtKB:A0A1B0GUA5",
  "gene_name": "Small integral membrane protein 32",
  "term_label": "Unknown molecular function"
}